follicle cell microvillus organization [GO:0032529] (BP) Also known as: follicle cell microvillus organisation, follicle cell microvillus organization and biogenesis Relationships: is a type of microvillus organization [GO:0032528] Regulation: regulated by regulation of follicle cell microvillus organization [GO:0032531] References: PMID:16507588 Sources: GOC:sart Definition: A process that is carried out at the cellular level which results in the assembly, arrangement of constituent parts, or disassembly of a microvillus on a follicle cell. A microvillus is a thin cylindrical membrane-covered projection on the surface of an animal cell containing a core bundle of actin filaments.